{
  "gene_symbol": "H2AC20",
  "gene_name": "Histone H2A type 2-C",
  "term_id": "GO:0000786",
  "term_label": "nucleosome",
  "gene": "UniProtKB:Q16777"
}